{
  "gene_symbol": "HSPA1A",
  "gene": "UniProtKB:P0DMV8",
  "term_label": "heat shock protein binding",
  "gene_name": "Heat shock 70 kDa protein 1A",
  "term_id": "GO:0031072"
}